{
  "term_id": "GO:0004478",
  "gene_name": "S-adenosylmethionine synthase isoform type-2",
  "gene": "UniProtKB:P31153",
  "term_label": "methionine adenosyltransferase activity",
  "gene_symbol": "MAT2A"
}